{
  "gene_symbol": "PIR",
  "gene_name": "Pirin",
  "gene": "UniProtKB:O00625",
  "term_id": "GO:0005634",
  "term_label": "nucleus"
}